{
  "gene": "UniProtKB:P01876",
  "term_label": "antigen binding",
  "gene_name": "Immunoglobulin heavy constant alpha 1",
  "term_id": "GO:0003823",
  "gene_symbol": "IGHA1"
}